{
  "term_label": "DNA repair",
  "gene_name": "CDK-activating kinase assembly factor MAT1",
  "term_id": "GO:0006281",
  "gene_symbol": "MNAT1",
  "gene": "UniProtKB:P51948"
}